{
  "gene_name": "Phospholipase A and acyltransferase 2",
  "term_id": "GO:0004623",
  "gene": "UniProtKB:Q9NWW9",
  "gene_symbol": "PLAAT2",
  "term_label": "phospholipase A2 activity"
}